{
  "gene": "UniProtKB:P15151",
  "gene_symbol": "PVR",
  "term_id": "GO:0005886",
  "gene_name": "Poliovirus receptor",
  "term_label": "plasma membrane"
}